{
  "term_id": "GO:0097228",
  "gene_symbol": "CATSPERZ",
  "term_label": "sperm principal piece",
  "gene": "UniProtKB:Q9NTU4",
  "gene_name": "Cation channel sperm-associated auxiliary subunit zeta"
}